{
  "term_label": "Unknown molecular function",
  "gene_name": "Tumor necrosis factor receptor superfamily member 21",
  "term_id": "UNKNOWN:0001",
  "gene_symbol": "TNFRSF21",
  "gene": "UniProtKB:O75509"
}